{
  "gene_symbol": "WDR45",
  "gene": "UniProtKB:Q9Y484",
  "gene_name": "WD repeat domain phosphoinositide-interacting protein 4",
  "term_id": "GO:0030674",
  "term_label": "protein-macromolecule adaptor activity"
}